{
  "term_id": "UNKNOWN:0002",
  "gene_symbol": "CSMD2",
  "term_label": "Unknown biological process",
  "gene_name": "CUB and sushi domain-containing protein 2",
  "gene": "UniProtKB:Q7Z408"
}